{
  "gene": "UniProtKB:Q13607",
  "term_id": "GO:0004984",
  "gene_symbol": "OR2F1",
  "term_label": "olfactory receptor activity",
  "gene_name": "Olfactory receptor 2F1"
}